{
  "gene_name": "Nectin-4",
  "gene": "UniProtKB:Q96NY8",
  "gene_symbol": "NECTIN4",
  "term_label": "plasma membrane",
  "term_id": "GO:0005886"
}